{
  "gene_symbol": "LINC00574",
  "term_id": "UNKNOWN:0002",
  "gene": "UniProtKB:Q9H8X3",
  "gene_name": "Putative uncharacterized protein LINC00574",
  "term_label": "Unknown biological process"
}